{
  "gene_symbol": "AVP",
  "gene": "UniProtKB:P01185",
  "gene_name": "Vasopressin-neurophysin 2-copeptin",
  "term_id": "GO:0002125",
  "term_label": "maternal aggressive behavior"
}